{
  "term_label": "metallocarboxypeptidase activity",
  "gene_symbol": "CPM",
  "gene": "UniProtKB:P14384",
  "term_id": "GO:0004181",
  "gene_name": "Carboxypeptidase M"
}